PDZ domain binding [GO:0030165] (molecular function) Definition: Binding to a PDZ domain of a protein, a domain found in diverse signaling proteins. Relationships: is a type of protein domain specific binding [GO:0019904] Also known as: DHR-domain binding, GLGF-domain binding Sources: GOC:go_curators, Pfam:PF00595